{
  "gene_symbol": "PPP3R2",
  "term_id": "GO:0019902",
  "gene_name": "Calcineurin subunit B type 2",
  "gene": "UniProtKB:Q96LZ3",
  "term_label": "phosphatase binding"
}